{
  "gene_name": "E-selectin",
  "gene_symbol": "SELE",
  "term_id": "GO:0050901",
  "term_label": "leukocyte tethering or rolling",
  "gene": "UniProtKB:P16581"
}